{
  "term_label": "synaptic vesicle recycling",
  "gene": "UniProtKB:Q14161",
  "term_id": "GO:0036465",
  "gene_name": "ARF GTPase-activating protein GIT2",
  "gene_symbol": "GIT2"
}